L-tryptophan import across plasma membrane [GO:1904272] (biological process) Definition: The directed movement of L-tryptophan from outside of a cell, across the plasma membrane and into the cytosol. References: PMID:21097500 Sources: GOC:TermGenie, GOC:kmv, GO_REF:0000075 Relationships: is a type of amino acid import across plasma membrane [GO:0089718]; is a type of GO:1904556